{
  "term_label": "Unknown cellular component",
  "gene_name": "Uncharacterized protein C15orf39",
  "term_id": "UNKNOWN:0003",
  "gene": "UniProtKB:Q6ZRI6",
  "gene_symbol": "C15orf39"
}